ent-isokaurene synthase activity [GO:0034281] (molecular function) Definition: Catalysis of the reaction: ent-copalyl diphosphate = ent-isokaurene + diphosphate. References: PMID:17141283 Relationships: is a type of terpene synthase activity [GO:0010333]